{
  "gene_symbol": "MEIS3",
  "term_id": "GO:0001228",
  "gene_name": "Homeobox protein Meis3",
  "gene": "UniProtKB:Q99687",
  "term_label": "DNA-binding transcription activator activity, RNA polymerase II-specific"
}